{
  "gene_symbol": "ZNF827",
  "term_id": "GO:0006355",
  "gene_name": "Zinc finger protein 827",
  "gene": "UniProtKB:Q17R98",
  "term_label": "regulation of DNA-templated transcription"
}